{
  "term_label": "Unknown biological process",
  "gene_name": "T cell receptor beta constant 2",
  "gene_symbol": "TRBC2",
  "term_id": "UNKNOWN:0002",
  "gene": "UniProtKB:A0A5B9"
}